UDP-2,3-diacylglucosamine hydrolase activity [GO:0008758] (molecular function) References: PMID:12000770 Sources: MetaCyc:LIPIDXSYNTHESIS-RXN Definition: Catalysis of the reaction: H2O + UDP-2,3-bis(3-hydroxymyristoyl)glucosamine = 2,3-bis(3-hydroxymyristoyl)-beta-D-glucosaminyl 1-phosphate + UMP. Relationships: is a type of pyrophosphatase activity [GO:0016462]